{
  "gene": "UniProtKB:Q8N4S9",
  "term_label": "apical plasma membrane",
  "term_id": "GO:0016324",
  "gene_symbol": "MARVELD2",
  "gene_name": "MARVEL domain-containing protein 2"
}